{
  "gene": "UniProtKB:Q92914",
  "gene_symbol": "FGF11",
  "term_label": "cytoplasm",
  "gene_name": "Fibroblast growth factor 11",
  "term_id": "GO:0005737"
}